synaptic membrane adhesion [GO:0099560] (biological process) Relationships: is a type of cell-cell adhesion [GO:0098609]; is part of synapse organization [GO:0050808] Regulation: regulated by regulation of synaptic membrane adhesion [GO:0099179] Also known as: synapse adhesion between pre- and post-synapse Sources: GOC:dos Definition: The attachment of presynaptic membrane to postsynaptic membrane via adhesion molecules that are at least partially embedded in the plasma membrane.